{
  "term_id": "GO:0045944",
  "gene": "UniProtKB:O60583",
  "gene_name": "Cyclin-T2",
  "term_label": "positive regulation of transcription by RNA polymerase II",
  "gene_symbol": "CCNT2"
}